mitotic spindle-templated microtubule nucleation [GO:0090221] (biological process) Relationships: is_a microtubule nucleation [GO:0007020] Definition: The 'de novo' formation of a microtubule, in which tubulin heterodimers form metastable oligomeric aggregates from within the mitotic spindle. Sources: GOC:ascb_2009, GOC:dph, GOC:tb